GCC codon-amino acid adaptor activity [GO:0033454] (molecular function) Sources: GOC:mah Also known as: alanine tRNA Definition: A triplet codon-amino acid adaptor activity that recognizes a GCC codon. Relationships: is a type of GO:0030533 Note: Note that in the standard genetic code, GCC codes for alanine.